{
  "gene_name": "Beta-1,3-galactosyl-O-glycosyl-glycoprotein beta-1,6-N-acetylglucosaminyltransferase 7",
  "term_id": "GO:0008375",
  "gene_symbol": "GCNT7",
  "term_label": "acetylglucosaminyltransferase activity",
  "gene": "UniProtKB:Q6ZNI0"
}